response to trehalose [GO:0010353] (biological process) Definition: Any process that results in a change in state or activity of a cell or an organism (in terms of movement, secretion, enzyme production, gene expression, etc.) as a result of a trehalose stimulus. References: PMID:17031512 Also known as: response to trehalose stimulus Relationships: is a type of GO:0034285 Subtypes: cellular response to trehalose stimulus [GO:0071327]